{
  "term_label": "cytoplasm",
  "gene_name": "RCC1 and BTB domain-containing protein 2",
  "gene_symbol": "RCBTB2",
  "gene": "UniProtKB:O95199",
  "term_id": "GO:0005737"
}